(1->3)-alpha-glucan metabolic process [GO:0070595] (biological process) Also known as: 1,3-alpha-glucan metabolic process, 1,3-alpha-glucan metabolism, alpha-1,3 glucan metabolic process, alpha-1,3 glucan metabolism Definition: The chemical reactions and pathways involving (1->3)-alpha-D-glucans, compounds composed of glucose residues linked by (1->3)-alpha-D-glucosidic bonds. Sources: GOC:mah Subtypes: GO:0070596, GO:0070597 Relationships: is a type of alpha-glucan metabolic process [GO:0030978]